{
  "gene": "UniProtKB:Q8NGX1",
  "gene_name": "Olfactory receptor 2T34",
  "term_label": "detection of chemical stimulus involved in sensory perception of smell",
  "gene_symbol": "OR2T34",
  "term_id": "GO:0050911"
}